{
  "gene_name": "Zinc finger protein with KRAB and SCAN domains 1",
  "gene_symbol": "ZKSCAN1",
  "gene": "UniProtKB:P17029",
  "term_id": "GO:0000981",
  "term_label": "DNA-binding transcription factor activity, RNA polymerase II-specific"
}